regulation of stomatal closure [GO:0090333] (biological process) Relationships: is a type of regulation of stomatal movement [GO:0010119]; regulates stomatal closure [GO:0090332] Sources: GOC:tb Definition: Any process that modulates the rate, frequency, or extent of stomatal closure. Stomatal closure is the process of closing of stomata, pores in the epidermis of leaves and stems bordered by two guard cells and serving in gas exchange.